positive regulation of mesoderm formation [GO:1905904] (biological process) Definition: Any process that activates or increases the frequency, rate or extent of mesoderm formation. References: PMID:23939491 Sources: GOC:BHF, GOC:BHF_miRNA, GOC:TermGenie, GOC:rph, GO_REF:0000058 Relationships: is a type of regulation of mesoderm formation [GO:1905902]; is a type of positive regulation of mesoderm development [GO:2000382]; RO_0002213 mesoderm formation [GO:0001707] Also known as: up regulation of mesoderm formation, up-regulation of mesoderm formation, upregulation of mesoderm formation, activation of mesoderm formation